{
  "term_label": "cytoplasm",
  "term_id": "GO:0005737",
  "gene": "UniProtKB:O00142",
  "gene_name": "Thymidine kinase 2, mitochondrial",
  "gene_symbol": "TK2"
}